{
  "gene_name": "Golgin subfamily A member 8M",
  "gene": "UniProtKB:H3BSY2",
  "term_id": "GO:0032580",
  "gene_symbol": "GOLGA8M",
  "term_label": "Golgi cisterna membrane"
}